{
  "gene_name": "Putative melanoma-associated antigen 5P",
  "gene": "UniProtKB:P43359",
  "term_id": "UNKNOWN:0001",
  "gene_symbol": "MAGEA5P",
  "term_label": "Unknown molecular function"
}